type Ib terminal bouton [GO:0061176] (cellular component) Sources: GOC:dph, GOC:mc Relationships: is a type of type I terminal bouton [GO:0061174] Definition: Terminal inflated portion of the axon of a glutamatergic neuron, containing the specialized apparatus necessary for the tonic release neurotransmitters that will induce the contraction of muscle. Type Ib terminal boutons are larger than type Is terminal boutons. Also known as: type Ib terminal button